{
  "gene_name": "Amyloid-beta A4 precursor protein-binding family A member 1",
  "gene_symbol": "APBA1",
  "term_label": "chemical synaptic transmission",
  "term_id": "GO:0007268",
  "gene": "UniProtKB:Q02410"
}